{
  "term_id": "GO:0006357",
  "gene_name": "Glucocorticoid receptor",
  "term_label": "regulation of transcription by RNA polymerase II",
  "gene_symbol": "NR3C1",
  "gene": "UniProtKB:P04150"
}